brain-derived neurotrophic factor receptor signaling pathway [GO:0031547] (biological process) Also known as: BDNF receptor signaling pathway, BDNF signalling pathway, brain-derived neurotrophic factor receptor signalling pathway Relationships: is a type of cell surface receptor protein tyrosine kinase signaling pathway [GO:0007169] Sources: GOC:mah Definition: The series of molecular signals generated as a consequence of a brain-derived neurotrophic factor receptor binding to one of its physiological ligands. Regulation: regulated by regulation of brain-derived neurotrophic factor receptor signaling pathway [GO:0031548]; negatively regulated by negative regulation of brain-derived neurotrophic factor receptor signaling pathway [GO:0031549]; positively regulated by positive regulation of brain-derived neurotrophic factor receptor signaling pathway [GO:0031550]